{
  "gene_name": "Perilipin-1",
  "gene_symbol": "PLIN1",
  "term_id": "UNKNOWN:0001",
  "term_label": "Unknown molecular function",
  "gene": "UniProtKB:O60240"
}